{
  "gene": "UniProtKB:Q13330",
  "term_id": "GO:0003714",
  "term_label": "transcription corepressor activity",
  "gene_symbol": "MTA1",
  "gene_name": "Metastasis-associated protein MTA1"
}